{
  "gene": "UniProtKB:Q9Y584",
  "gene_symbol": "TIMM22",
  "gene_name": "Mitochondrial import inner membrane translocase subunit Tim22",
  "term_id": "GO:0008320",
  "term_label": "protein transmembrane transporter activity"
}